{
  "gene_symbol": "UBXN2B",
  "term_label": "nuclear membrane reassembly",
  "gene": "UniProtKB:Q14CS0",
  "gene_name": "UBX domain-containing protein 2B",
  "term_id": "GO:0031468"
}